{
  "gene": "UniProtKB:P09382",
  "term_label": "Unknown biological process",
  "gene_name": "Galectin-1",
  "gene_symbol": "LGALS1",
  "term_id": "UNKNOWN:0002"
}